{
  "term_label": "Unknown molecular function",
  "gene_name": "Proteasome subunit alpha type-4",
  "gene": "UniProtKB:P25789",
  "gene_symbol": "PSMA4",
  "term_id": "UNKNOWN:0001"
}